regulation of midbrain dopaminergic neuron differentiation [GO:1904956] (biological process) Relationships: is a type of regulation of dopaminergic neuron differentiation [GO:1904338]; regulates midbrain dopaminergic neuron differentiation [GO:1904948] References: PMID:21347250 Sources: GOC:PARL, GOC:TermGenie, GOC:bf, GO_REF:0000058 Subtypes: negative regulation of midbrain dopaminergic neuron differentiation [GO:1904957], positive regulation of midbrain dopaminergic neuron differentiation [GO:1904958] Definition: Any process that modulates the frequency, rate or extent of midbrain dopaminergic neuron differentiation. Also known as: regulation of DA neurogenesis from midbrain floor plate, regulation of mDA neuron differentiation, regulation of midbrain DA neurogenesis, regulation of midbrain dopaminergic neuron production